{
  "gene": "UniProtKB:O75311",
  "term_id": "GO:0005231",
  "gene_symbol": "GLRA3",
  "term_label": "excitatory extracellular ligand-gated monoatomic ion channel activity",
  "gene_name": "Glycine receptor subunit alpha-3"
}